meiosis II nuclear membrane reassembly [GO:0051335] (biological process) Relationships: is a type of GO:0051333; is part of meiosis II [GO:0007135] Sources: GOC:ai Definition: The reformation of the nuclear membrane during meiosis II. Also known as: meiosis II nuclear envelope reassembly